{
  "term_id": "GO:0005871",
  "gene_name": "Kinesin-like protein KIF2C",
  "gene": "UniProtKB:Q99661",
  "term_label": "kinesin complex",
  "gene_symbol": "KIF2C"
}